vesicle targeting, trans-Golgi to periciliary membrane compartment [GO:0097712] (biological process) References: PMID:20106869, PMID:23351793, PMID:24814148, PMID:26485645 Sources: GOC:cilia Relationships: is a type of vesicle targeting, to, from or within Golgi [GO:0048199]; BFO_0000050 cilium assembly [GO:0060271] Definition: The process in which vesicles formed at the trans-Golgi network are directed to the plasma membrane surrounding the base of the cilium, including the ciliary pocket, mediated by molecules at the vesicle membrane and target membrane surfaces.